adult heart development [GO:0007512] (biological process) Sources: GOC:bf Also known as: adult cardiac development Relationships: is_a heart development [GO:0007507] Definition: The process whose specific outcome is the progression of the adult heart over time, from its formation to the mature structure.